{
  "term_label": "nucleolus",
  "gene_symbol": "AOPEP",
  "gene": "UniProtKB:Q8N6M6",
  "gene_name": "Aminopeptidase O",
  "term_id": "GO:0005730"
}